{
  "gene_name": "Cytoskeleton-associated protein 4",
  "gene_symbol": "CKAP4",
  "gene": "UniProtKB:Q07065",
  "term_label": "Unknown molecular function",
  "term_id": "UNKNOWN:0001"
}